{
  "term_label": "cellular response to cadmium ion",
  "gene": "UniProtKB:P13640",
  "gene_symbol": "MT1G",
  "term_id": "GO:0071276",
  "gene_name": "Metallothionein-1G"
}